growth plate cartilage chondrocyte development [GO:0003431] (biological process) Sources: GOC:ascb_2009, GOC:dph, GOC:tb Relationships: is a type of GO:0003433; BFO_0000050 growth plate cartilage chondrocyte differentiation [GO:0003418] Definition: The progression of a growth plate cartilage chondrocyte over time from after its fate commitment to the mature cell.